regulation of estrogen secretion [GO:2000861] (biological process) Relationships: is_a regulation of steroid hormone secretion [GO:2000831]; regulates estrogen secretion [GO:0035937] Sources: GOC:sl Also known as: regulation of oestrogen secretion Subtypes: negative regulation of estrogen secretion [GO:2000862], positive regulation of estrogen secretion [GO:2000863] Definition: Any process that modulates the frequency, rate or extent of estrogen secretion.